MHC protein complex binding [GO:0023023] (molecular function) Sources: GOC:mtg_signal, GOC:vw Relationships: is a type of protein-containing complex binding [GO:0044877] Subtypes: MHC class I protein complex binding [GO:0023024], MHC class Ib protein complex binding [GO:0023025], MHC class II protein complex binding [GO:0023026] Definition: Binding to a major histocompatibility complex.